positive regulation of nucleotide biosynthetic process [GO:0030810] (biological process) Relationships: is a type of GO:0009891; is a type of regulation of nucleotide biosynthetic process [GO:0030808]; is a type of positive regulation of nucleotide metabolic process [GO:0045981]; positively regulates GO:0009165 Also known as: positive regulation of nucleotide anabolism, positive regulation of nucleotide biosynthesis, positive regulation of nucleotide formation, positive regulation of nucleotide synthesis, up regulation of nucleotide biosynthetic process, up-regulation of nucleotide biosynthetic process, upregulation of nucleotide biosynthetic process, activation of nucleotide biosynthetic process, stimulation of nucleotide biosynthetic process Subtypes: positive regulation of purine nucleotide biosynthetic process [GO:1900373], positive regulation of pyrimidine nucleotide biosynthetic process [GO:1900399] Definition: Any process that activates or increases the frequency, rate or extent of the chemical reactions and pathways resulting in the formation of nucleotides. Sources: GOC:mah